{
  "term_label": "nucleus",
  "term_id": "GO:0005634",
  "gene": "UniProtKB:Q9Y4X0",
  "gene_symbol": "AMMECR1",
  "gene_name": "Nuclear protein AMMECR1"
}